{
  "term_label": "plasma membrane",
  "gene": "UniProtKB:Q8N8Z6",
  "gene_symbol": "DCBLD1",
  "term_id": "GO:0005886",
  "gene_name": "Discoidin, CUB and LCCL domain-containing protein 1"
}